{
  "gene": "UniProtKB:Q9H4M9",
  "gene_symbol": "EHD1",
  "term_id": "GO:0005769",
  "term_label": "early endosome",
  "gene_name": "EH domain-containing protein 1"
}